localization [GO:0051179] (biological process) Relationships: is a type of biological_process [GO:0008150] Sources: GOC:ai, GOC:dos Also known as: establishment and maintenance of localization, establishment and maintenance of position, localisation, establishment and maintenance of cellular component location, establishment and maintenance of substance location, establishment and maintenance of substrate location, single organism localization, single-organism localization Subtypes: macromolecule localization [GO:0033036], GO:0035732, GO:0051234, maintenance of location [GO:0051235], organelle localization [GO:0051640], GO:0051641, localization of cell [GO:0051674], GO:0061842, receptor localization to synapse [GO:0097120] Definition: Any process in which a cell, a substance, or a cellular entity, such as a protein complex or organelle, is transported, tethered to or otherwise maintained in a specific location. In the case of substances, localization may also be achieved via selective degradation. Regulation: regulated by regulation of localization [GO:0032879]